{
  "gene": "UniProtKB:P0DUB6",
  "gene_name": "Alpha-amylase 1A",
  "term_id": "GO:0004556",
  "gene_symbol": "AMY1A",
  "term_label": "alpha-amylase activity"
}